{
  "term_id": "GO:0005656",
  "gene_symbol": "WDR18",
  "gene": "UniProtKB:Q9BV38",
  "term_label": "nuclear pre-replicative complex",
  "gene_name": "WD repeat-containing protein 18"
}